beta-mannosidase activity [GO:0004567] (molecular function) Sources: EC:3.2.1.25 Relationships: is a type of GO:0015923 Also known as: beta-D-mannosidase activity, beta-D-mannoside mannohydrolase activity, beta-mannoside mannohydrolase activity, exo-beta-D-mannanase activity, mannanase activity, mannase activity Subtypes: mannan endo-1,4-beta-mannosidase activity [GO:0016985], mannosylglycoprotein endo-beta-mannosidase activity [GO:0033947] Definition: Catalysis of the hydrolysis of terminal, non-reducing beta-D-mannose residues in beta-D-mannosides.